acylglycerol acyl-chain remodeling [GO:0036155] (biological process) Also known as: acylglycerol acyl-chain remodelling, glyceride acyl-chain remodeling Relationships: is a type of acylglycerol metabolic process [GO:0006639] Definition: Remodeling the acyl chains of an acylglycerol, through sequential deacylation and re-acylation reactions, to generate an acylglycerol containing different types of fatty acid acyl chains. Subtypes: triglyceride acyl-chain remodeling [GO:0036153], GO:0036154 References: PMID:15364929 Sources: GOC:mw